{
  "gene_name": "Progesterone receptor",
  "term_label": "nuclear receptor activity",
  "gene": "UniProtKB:P06401",
  "gene_symbol": "PGR",
  "term_id": "GO:0004879"
}